{
  "term_label": "ubiquitin protein ligase activity",
  "gene_name": "Probable E3 ubiquitin-protein ligase HERC4",
  "gene_symbol": "HERC4",
  "gene": "UniProtKB:Q5GLZ8",
  "term_id": "GO:0061630"
}